sphingomyelin metabolic process [GO:0006684] (biological process) Sources: ISBN:0198506732 Subtypes: sphingomyelin catabolic process [GO:0006685], sphingomyelin biosynthetic process [GO:0006686] Relationships: is a type of GO:0006644; is a type of sphingolipid metabolic process [GO:0006665]; is a type of amide metabolic process [GO:0043603] Definition: The chemical reactions and pathways involving sphingomyelin, N-acyl-4-sphingenyl-1-O-phosphorylcholine, any of a class of phospholipids in which the amino group of sphingosine is in amide linkage with one of several fatty acids, while the terminal hydroxyl group of sphingosine is esterified to phosphorylcholine. Also known as: sphingomyelin metabolism